catecholamine transport [GO:0051937] (biological process) Relationships: is a type of monoamine transport [GO:0015844]; is a type of organic hydroxy compound transport [GO:0015850] Sources: GOC:ai, ISBN:0198506732 Definition: The directed movement of catecholamines, a group of physiologically important biogenic amines that possess a catechol (3,4-dihydroxyphenyl) nucleus and are derivatives of 3,4-dihydroxyphenylethylamine. Subtypes: dopamine transport [GO:0015872], norepinephrine transport [GO:0015874], epinephrine transport [GO:0048241], catecholamine secretion [GO:0050432], catecholamine uptake [GO:0090493]